{
  "gene_name": "Probable G-protein coupled receptor 32",
  "term_label": "positive regulation of cytosolic calcium ion concentration",
  "term_id": "GO:0007204",
  "gene": "UniProtKB:O75388",
  "gene_symbol": "GPR32"
}